{
  "term_label": "sterol metabolic process",
  "gene_symbol": "UGT1A9",
  "term_id": "GO:0016125",
  "gene_name": "UDP-glucuronosyltransferase 1A9",
  "gene": "UniProtKB:O60656"
}